regulation of cell cycle phase transition [GO:1901987] (biological process) Subtypes: GO:1901976, GO:1901988, positive regulation of cell cycle phase transition [GO:1901989], regulation of mitotic cell cycle phase transition [GO:1901990], GO:1901993, regulation of metaphase/anaphase transition of cell cycle [GO:1902099], regulation of cell cycle G2/M phase transition [GO:1902749], GO:1902806 Relationships: is a type of regulation of cell cycle process [GO:0010564]; regulates GO:0044770 Also known as: cell cycle control, regulation of cell cycle transition References: PMID:22841721 Sources: GOC:TermGenie, GOC:mtg_cell_cycle Definition: Any process that modulates the frequency, rate or extent of cell cycle phase transition.